{
  "gene_symbol": "CNTN3",
  "term_label": "Unknown biological process",
  "gene_name": "Contactin-3",
  "gene": "UniProtKB:Q9P232",
  "term_id": "UNKNOWN:0002"
}